positive regulation of nucleotide-binding oligomerization domain containing 2 signaling pathway [GO:0070434] (biological process) Also known as: positive regulation of NOD2 signaling pathway, positive regulation of nucleotide-binding oligomerization domain containing 2 signalling pathway Definition: Any process that activates or increases the frequency, rate, or extent of the nucleotide-binding oligomerization domain containing 2 (NOD2) pathway. Sources: GOC:add Relationships: is a type of positive regulation of nucleotide-binding domain, leucine rich repeat containing receptor signaling pathway [GO:0070426]; is a type of regulation of nucleotide-binding oligomerization domain containing 2 signaling pathway [GO:0070432]; positively regulates GO:0070431